anandamide epoxidase activity [GO:0062186] (molecular function) Subtypes: GO:0062187, anandamide 11,12 epoxidase activity [GO:0062188], anandamide 14,15 epoxidase activity [GO:0062189] Also known as: arachidonoylethanolamide epoxidase activity References: PMID:21289075 Relationships: is a type of GO:0016709 Definition: Catalysis of the epoxidation of double bonds of the arachidonoyl moiety of anandamide.